{
  "gene": "UniProtKB:P37837",
  "term_label": "pentose-phosphate shunt, non-oxidative branch",
  "gene_name": "Transaldolase",
  "term_id": "GO:0009052",
  "gene_symbol": "TALDO1"
}